{
  "term_id": "GO:0006511",
  "gene_name": "E3 ubiquitin-protein ligase HUWE1",
  "term_label": "ubiquitin-dependent protein catabolic process",
  "gene": "UniProtKB:Q7Z6Z7",
  "gene_symbol": "HUWE1"
}